{
  "gene_symbol": "ZNF343",
  "term_id": "GO:0000981",
  "gene_name": "Zinc finger protein 343",
  "gene": "UniProtKB:Q6P1L6",
  "term_label": "DNA-binding transcription factor activity, RNA polymerase II-specific"
}